{
  "term_id": "UNKNOWN:0002",
  "gene_symbol": "FAM219A",
  "gene_name": "Protein FAM219A",
  "term_label": "Unknown biological process",
  "gene": "UniProtKB:Q8IW50"
}